{
  "gene_name": "Junctophilin-4",
  "gene": "UniProtKB:Q96JJ6",
  "term_id": "GO:0005789",
  "gene_symbol": "JPH4",
  "term_label": "endoplasmic reticulum membrane"
}